{
  "term_label": "putrescine binding",
  "term_id": "GO:0019810",
  "gene_name": "S-adenosylmethionine decarboxylase proenzyme",
  "gene_symbol": "AMD1",
  "gene": "UniProtKB:P17707"
}